{
  "gene_name": "Syntaxin-7",
  "gene_symbol": "STX7",
  "gene": "UniProtKB:O15400",
  "term_label": "intracellular protein transport",
  "term_id": "GO:0006886"
}